{
  "term_id": "GO:0004930",
  "gene_symbol": "ADGRF3",
  "term_label": "G protein-coupled receptor activity",
  "gene_name": "Adhesion G-protein coupled receptor F3",
  "gene": "UniProtKB:Q8IZF5"
}